{
  "gene": "UniProtKB:A0A075B7D8",
  "gene_symbol": "IGHV3OR15-7",
  "term_label": "antigen binding",
  "gene_name": "Immunoglobulin heavy variable 3_OR15-7 (pseudogene) (Fragment)",
  "term_id": "GO:0003823"
}